{
  "gene_name": "Zinc finger protein 440",
  "gene": "UniProtKB:Q8IYI8",
  "term_label": "RNA polymerase II transcription regulatory region sequence-specific DNA binding",
  "gene_symbol": "ZNF440",
  "term_id": "GO:0000977"
}